2-(omega-methylthio)alkylmalate dehydratase activity [GO:0120528] (molecular function) Definition: Catalysis of the reactions: a 2-(omega-methylsulfanyl)alkylmalate = a 2-(omega-methylsulfanyl)alkylmaleate + H2O and a 3-(omega-methylsulfanyl)alkylmalate = a 2-(omega-methylsulfanyl)alkylmaleate + H2O. Relationships: is a type of GO:0016836 Sources: EC:4.2.1.170